{
  "gene_symbol": "ARPC4",
  "gene_name": "Actin-related protein 2_3 complex subunit 4",
  "gene": "UniProtKB:P59998",
  "term_id": "GO:0005885",
  "term_label": "Arp2/3 protein complex"
}